{
  "term_id": "GO:0007165",
  "gene": "UniProtKB:Q7Z7M0",
  "gene_name": "Multiple epidermal growth factor-like domains protein 8",
  "gene_symbol": "MEGF8",
  "term_label": "signal transduction"
}